{
  "term_label": "phosphatidylinositol phosphate binding",
  "gene": "UniProtKB:Q969T3",
  "gene_symbol": "SNX21",
  "term_id": "GO:1901981",
  "gene_name": "Sorting nexin-21"
}